error-prone translesion synthesis [GO:0042276] (biological process) Definition: The conversion of DNA-damage induced single-stranded gaps into large molecular weight DNA after replication by using a specialized DNA polymerase or replication complex to insert a defined nucleotide across the lesion. This process does not remove the replication-blocking lesions and causes an increase in the endogenous mutation level. For example, in E. coli, a low fidelity DNA polymerase, pol V, copies lesions that block replication fork progress. This produces mutations specifically targeted to DNA template damage sites, but it can also produce mutations at undamaged sites. References: PMID:11485998 Sources: GOC:elh, GOC:jl Also known as: mutagenic PRR, error-prone postreplication DNA repair, mutagenic postreplication DNA repair Relationships: is a type of translesion synthesis [GO:0019985] Regulation: regulated by GO:1904331; negatively regulated by negative regulation of error-prone translesion synthesis [GO:1904332]; positively regulated by positive regulation of error-prone translesion synthesis [GO:1904333]